{
  "term_label": "regulation of cell projection organization",
  "gene_name": "Ermin",
  "term_id": "GO:0031344",
  "gene": "UniProtKB:Q8TAM6",
  "gene_symbol": "ERMN"
}